{
  "term_id": "UNKNOWN:0001",
  "gene_name": "Probable non-functional immunoglobulin kappa variable 3-7",
  "term_label": "Unknown molecular function",
  "gene": "UniProtKB:A0A075B6H7",
  "gene_symbol": "IGKV3-7"
}